positive regulation of cardiolipin metabolic process [GO:1900210] (biological process) Also known as: activation of cardiolipin metabolism, positive regulation of cardiolipin metabolism, up regulation of cardiolipin metabolic process, up regulation of cardiolipin metabolism, up-regulation of cardiolipin metabolic process, up-regulation of cardiolipin metabolism, upregulation of cardiolipin metabolic process, upregulation of cardiolipin metabolism, activation of cardiolipin metabolic process, activation of diphosphatidylglycerol metabolic process, activation of diphosphatidylglycerol metabolism, positive regulation of diphosphatidylglycerol metabolic process, positive regulation of diphosphatidylglycerol metabolism, up regulation of diphosphatidylglycerol metabolic process, up regulation of diphosphatidylglycerol metabolism, up-regulation of diphosphatidylglycerol metabolic process, up-regulation of diphosphatidylglycerol metabolism, upregulation of diphosphatidylglycerol metabolic process, upregulation of diphosphatidylglycerol metabolism Definition: Any process that activates or increases the frequency, rate or extent of cardiolipin metabolic process. Relationships: is a type of GO:1900208; is_a positive regulation of phospholipid metabolic process [GO:1903727]; positively regulates cardiolipin metabolic process [GO:0032048] Sources: GOC:TermGenie